{
  "term_label": "Unknown biological process",
  "term_id": "UNKNOWN:0002",
  "gene_symbol": "NPIPA2",
  "gene": "UniProtKB:E9PIF3",
  "gene_name": "Nuclear pore complex-interacting protein family member A2"
}